{
  "gene_name": "TBC1 domain family member 8",
  "gene_symbol": "TBC1D8",
  "term_label": "Unknown biological process",
  "term_id": "UNKNOWN:0002",
  "gene": "UniProtKB:O95759"
}